{
  "term_label": "formation of translation preinitiation complex",
  "term_id": "GO:0001731",
  "gene_symbol": "MCTS1",
  "gene_name": "Malignant T-cell-amplified sequence 1",
  "gene": "UniProtKB:Q9ULC4"
}